{
  "term_label": "Unknown molecular function",
  "gene_name": "DDB1- and CUL4-associated factor 8",
  "term_id": "UNKNOWN:0001",
  "gene": "UniProtKB:Q5TAQ9",
  "gene_symbol": "DCAF8"
}